{
  "term_id": "UNKNOWN:0002",
  "gene_name": "Leucine-rich repeat and transmembrane domain-containing protein 2",
  "gene_symbol": "LRTM2",
  "gene": "UniProtKB:Q8N967",
  "term_label": "Unknown biological process"
}